{
  "gene": "UniProtKB:Q86T20",
  "term_id": "UNKNOWN:0001",
  "gene_symbol": "SMIM29",
  "gene_name": "Small integral membrane protein 29",
  "term_label": "Unknown molecular function"
}